regulation of inner ear auditory receptor cell differentiation [GO:0045607] (biological process) Relationships: is a type of regulation of epidermal cell differentiation [GO:0045604]; is a type of GO:2000980; regulates inner ear auditory receptor cell differentiation [GO:0042491] Subtypes: regulation of inner ear auditory receptor cell fate specification [GO:0042669], negative regulation of inner ear auditory receptor cell differentiation [GO:0045608], GO:0045609 Sources: GOC:go_curators Also known as: regulation of auditory hair cell differentiation, regulation of auditory receptor cell differentiation Definition: Any process that modulates the frequency, rate or extent of auditory hair cell differentiation.